adenylyl-sulfate reductase (glutathione) activity [GO:0033741] (molecular function) Relationships: is a type of oxidoreductase activity, acting on a sulfur group of donors, disulfide as acceptor [GO:0016671] Also known as: plant-type 5'-adenylylsulfate reductase activity, 5'-adenylylsulfate reductase activity, AMP,sulfite:glutathione-disulfide oxidoreductase (adenosine-5'-phosphosulfate-forming) activity, AMP,sulfite:oxidized-glutathione oxidoreductase (adenosine-5'-phosphosulfate-forming) activity Definition: Catalysis of the reaction: AMP + glutathione disulfide + H+ + sulfite = 5'-adenylyl sulfate + 2 glutathione. Sources: EC:1.8.4.9, RHEA:14141